{
  "term_id": "GO:0005576",
  "gene": "UniProtKB:Q99944",
  "term_label": "extracellular region",
  "gene_name": "Epidermal growth factor-like protein 8",
  "gene_symbol": "EGFL8"
}